(3R)-2'-hydroxyisoflavanone reductase (NADP+) activity [GO:0140860] (molecular function) References: PMID:7625843 Sources: RHEA:56284 Also known as: vestitone reductase activity Relationships: is a type of oxidoreductase activity, acting on the CH-OH group of donors, NAD or NADP as acceptor [GO:0016616] Definition: Catalysis of the reaction: a (3R,4R)-4,2'-dihydroxyisoflavan + NADP+ = a (3R)-2'-hydroxyisoflavanone + H+ + NADPH.